{
  "term_label": "nucleus",
  "gene": "UniProtKB:O60506",
  "term_id": "GO:0005634",
  "gene_symbol": "SYNCRIP",
  "gene_name": "Heterogeneous nuclear ribonucleoprotein Q"
}